{
  "gene_symbol": "HPX",
  "term_label": "heme metabolic process",
  "gene": "UniProtKB:P02790",
  "gene_name": "Hemopexin",
  "term_id": "GO:0042168"
}